{
  "term_id": "GO:0016192",
  "gene": "UniProtKB:Q96JC1",
  "gene_symbol": "VPS39",
  "gene_name": "Vam6_Vps39-like protein",
  "term_label": "vesicle-mediated transport"
}